isoprene biosynthetic process [GO:0043612] (biological process) Definition: The chemical reactions and pathways resulting in the formation of isoprene, C5H8. Relationships: is a type of isoprene metabolic process [GO:0043611]; is a type of GO:0046246; is a type of olefin biosynthetic process [GO:1900674] Regulation: regulated by regulation of isoprene biosynthetic process [GO:1900947]; negatively regulated by negative regulation of isoprene biosynthetic process [GO:1900948]; positively regulated by positive regulation of isoprene biosynthetic process [GO:1900949] Also known as: 2-methyl-1,3-butadiene biosynthesis, 2-methyl-1,3-butadiene biosynthetic process, hemiterpene biosynthesis, hemiterpene biosynthetic process Sources: GOC:jl